{
  "gene": "UniProtKB:P84074",
  "gene_symbol": "HPCA",
  "term_label": "Unknown cellular component",
  "term_id": "UNKNOWN:0003",
  "gene_name": "Neuron-specific calcium-binding protein hippocalcin"
}